{
  "gene_symbol": "Q96NJ1",
  "gene_name": "Uncharacterized protein FLJ30774",
  "gene": "UniProtKB:Q96NJ1",
  "term_id": "UNKNOWN:0001",
  "term_label": "Unknown molecular function"
}